{
  "gene_symbol": "GRIK5",
  "term_id": "GO:1904315",
  "gene_name": "Glutamate receptor ionotropic, kainate 5",
  "term_label": "transmitter-gated monoatomic ion channel activity involved in regulation of postsynaptic membrane potential",
  "gene": "UniProtKB:Q16478"
}